methanethiol oxidase activity [GO:0018549] (molecular function) Also known as: (MM)-oxidase activity, MT-oxidase activity, methanethiol:oxygen oxidoreductase activity, methyl mercaptan oxidase activity, methylmercaptan oxidase activity Sources: EC:1.8.3.4 Relationships: is a type of GO:0016670 Definition: Catalysis of the reaction: methanethiol + O2 + H2O = formaldehyde + hydrogen sulfide + hydrogen peroxide.